{
  "term_id": "UNKNOWN:0001",
  "term_label": "Unknown molecular function",
  "gene_name": "Intraflagellar transport protein 52 homolog",
  "gene": "UniProtKB:Q9Y366",
  "gene_symbol": "IFT52"
}